hexuronide transmembrane transport [GO:0015778] (biological process) Relationships: is a type of carbohydrate transmembrane transport [GO:0034219] Also known as: hexuronide transport Definition: The directed movement of hexuronide across a membrane. Hexuronides are any compound formed by combination of glycosidic linkage of a hydroxy compound (e.g. an alcohol or a saccharide) with the anomeric carbon atom of a hexuronate. Sources: GOC:ai